{
  "gene_symbol": "ZNF217",
  "gene": "UniProtKB:O75362",
  "gene_name": "Zinc finger protein 217",
  "term_id": "GO:0000978",
  "term_label": "RNA polymerase II cis-regulatory region sequence-specific DNA binding"
}